{
  "gene": "UniProtKB:Q9P244",
  "gene_symbol": "LRFN1",
  "term_label": "Unknown biological process",
  "gene_name": "Leucine-rich repeat and fibronectin type III domain-containing protein 1",
  "term_id": "UNKNOWN:0002"
}